{
  "gene_symbol": "APOBEC1",
  "gene": "UniProtKB:P41238",
  "gene_name": "C-U-editing enzyme APOBEC-1",
  "term_id": "GO:0003723",
  "term_label": "RNA binding"
}